{
  "gene": "UniProtKB:P05155",
  "term_label": "serine-type endopeptidase inhibitor activity",
  "gene_name": "Plasma protease C1 inhibitor",
  "term_id": "GO:0004867",
  "gene_symbol": "SERPING1"
}